endothelin receptor activity [GO:0004962] (molecular function) Relationships: is a type of G protein-coupled peptide receptor activity [GO:0008528]; is part of endothelin receptor signaling pathway [GO:0086100] Also known as: endothelin-A receptor activity, endothelin-B receptor activity Sources: GOC:bf, GOC:dph, GOC:signaling, IUPHAR_GPCR:1283, IUPHAR_RECEPTOR:2263 Definition: Combining with endothelin and transmitting the signal across the membrane by activating an associated G-protein; promotes the exchange of GDP for GTP on the alpha subunit of a heterotrimeric G-protein complex.